{
  "term_id": "GO:0005813",
  "gene_symbol": "CEP57",
  "gene": "UniProtKB:Q86XR8",
  "gene_name": "Centrosomal protein of 57 kDa",
  "term_label": "centrosome"
}